{
  "gene_name": "Testis-specific Y-encoded protein 2",
  "gene_symbol": "TSPY2",
  "term_label": "histone binding",
  "term_id": "GO:0042393",
  "gene": "UniProtKB:A6NKD2"
}